receptor signaling protein tyrosine kinase activator activity [GO:0030298] (MF) Also known as: receptor signalling protein tyrosine kinase activator activity Sources: GOC:mah Definition: Binds to and increases the activity of a receptor signaling protein tyrosine kinase. Relationships: is a type of protein tyrosine kinase activator activity [GO:0030296]